{
  "gene": "UniProtKB:P51965",
  "term_label": "ISG15-protein conjugation",
  "gene_name": "Ubiquitin-conjugating enzyme E2 E1",
  "term_id": "GO:0032020",
  "gene_symbol": "UBE2E1"
}